{
  "term_label": "BLOC-1 complex",
  "gene_symbol": "BLOC1S6",
  "gene_name": "Biogenesis of lysosome-related organelles complex 1 subunit 6",
  "term_id": "GO:0031083",
  "gene": "UniProtKB:Q9UL45"
}